cytoplasmic side of cis-Golgi network membrane [GO:0140179] (cellular component) Definition: The leaflet of the membrane bilayer of the cis-Golgi network faces the cytoplasm and is where interactions with cytosolic proteins occur, including those for vesicle tethering, fusion, and Golgi-associated trafficking activities. References: PMID:1747103, PMID:23913272, PMID:34080016, PMID:34597626 Relationships: is_a cytoplasmic side of membrane [GO:0098562]; BFO_0000050 GO:0033106